protoporphyrinogen IX biosynthetic process from glutamate [GO:0019353] (biological process) Also known as: protoporphyrinogen IX anabolism from glutamate, protoporphyrinogen IX formation from glutamate, protoporphyrinogen IX synthesis from glutamate Relationships: is a type of protoporphyrinogen IX biosynthetic process [GO:0006782]; is a type of GO:0033526 References: PMID:32976912 Definition: The chemical reactions and pathways resulting in the formation of protoporphyrinogen IX from other compounds, including glutamate.